2',3'-cyclic GMP-AMP binding [GO:0061507] (molecular function) Definition: Binding to 2',3' cyclic GMP-AMP (cGAMP) nucleotide, a cyclic purine dinucleotide that consists of AMP and GMP units cyclized via 2',5' and 3',5' linkages. References: PMID:23258412, PMID:23910378 Sources: GOC:dph Relationships: is a type of adenyl ribonucleotide binding [GO:0032559]; is a type of guanyl ribonucleotide binding [GO:0032561]; is a type of GO:0043168; is a type of cyclic GMP-AMP binding [GO:0140702] Also known as: cyclic-GMP-AMP binding, 2',3' cGAMP binding, 2',3' cyclic GAMP binding, 2',3'-cGAMP binding, 2',3'-cyclic GAMP binding, 2',5-3',5'-cyclic GMP-AMP binding, c[G(2',5')pA(3',5')p] binding